positive regulation of dense core granule exocytosis [GO:1905415] (BP) Definition: Any process that activates or increases the frequency, rate or extent of dense core granule exocytosis. References: PMID:18468511 Sources: GOC:PARL, GOC:TermGenie, GOC:bf, GO_REF:0000058 Also known as: positive regulation of dense core vesicle exocytosis, up regulation of dense core granule exocytosis, up regulation of dense core vesicle exocytosis, up-regulation of dense core granule exocytosis, up-regulation of dense core vesicle exocytosis, upregulation of dense core granule exocytosis, upregulation of dense core vesicle exocytosis, activation of dense core granule exocytosis, activation of dense core vesicle exocytosis Relationships: is a type of positive regulation of calcium ion-dependent exocytosis [GO:0045956]; is a type of regulation of dense core granule exocytosis [GO:1905413]; positively regulates dense core granule exocytosis [GO:1990504]